{
  "term_id": "UNKNOWN:0002",
  "term_label": "Unknown biological process",
  "gene": "UniProtKB:Q96NL0",
  "gene_symbol": "RUNDC3B",
  "gene_name": "RUN domain-containing protein 3B"
}